{
  "term_id": "UNKNOWN:0002",
  "gene": "UniProtKB:Q9BSJ8",
  "term_label": "Unknown biological process",
  "gene_symbol": "ESYT1",
  "gene_name": "Extended synaptotagmin-1"
}